{
  "term_label": "plasma membrane",
  "gene_name": "Interferon-induced transmembrane protein 1",
  "gene_symbol": "IFITM1",
  "gene": "UniProtKB:P13164",
  "term_id": "GO:0005886"
}